{
  "gene": "UniProtKB:Q6KB66",
  "term_label": "keratinization",
  "gene_name": "Keratin, type II cytoskeletal 80",
  "gene_symbol": "KRT80",
  "term_id": "GO:0031424"
}